regulation of protection from non-homologous end joining at telomere [GO:1905764] (BP) Subtypes: negative regulation of protection from non-homologous end joining at telomere [GO:1905765], positive regulation of protection from non-homologous end joining at telomere [GO:1905766] Relationships: is a type of regulation of telomere capping [GO:1904353]; is_a regulation of telomere maintenance in response to DNA damage [GO:1904505]; regulates GO:0031848 References: PMID:14690602 Sources: GOC:BHF, GOC:BHF_telomere, GOC:TermGenie, GOC:nc, GO_REF:0000058 Also known as: regulation of protection from NHEJ-mediated telomere fusion Definition: Any process that modulates the frequency, rate or extent of protection from non-homologous end joining at telomere.